{
  "term_id": "GO:0060261",
  "term_label": "positive regulation of transcription initiation by RNA polymerase II",
  "gene_name": "Mediator of RNA polymerase II transcription subunit 18",
  "gene_symbol": "MED18",
  "gene": "UniProtKB:Q9BUE0"
}